{
  "gene_symbol": "FASTKD5",
  "term_label": "mitochondrial RNA processing",
  "gene": "UniProtKB:Q7L8L6",
  "gene_name": "FAST kinase domain-containing protein 5, mitochondrial",
  "term_id": "GO:0000963"
}